sulfathiazole transmembrane transport [GO:1902599] (biological process) Definition: The directed movement of sulfathiazole across a membrane. Sources: GOC:TermGenie, GOC:pr, GO_REF:0000069 Also known as: sulfathiazole transport, sulphathiazole transport Relationships: is a type of amide transport [GO:0042886]; is a type of azole transmembrane transport [GO:0045117]; is a type of sulfur compound transport [GO:0072348]